{
  "gene_symbol": "PAK5",
  "term_id": "GO:0035556",
  "term_label": "intracellular signal transduction",
  "gene": "UniProtKB:Q9P286",
  "gene_name": "Serine_threonine-protein kinase PAK 5"
}